{
  "term_label": "Unknown cellular component",
  "term_id": "UNKNOWN:0003",
  "gene": "UniProtKB:Q13370",
  "gene_symbol": "PDE3B",
  "gene_name": "cGMP-inhibited 3',5'-cyclic phosphodiesterase 3B"
}